{
  "gene": "UniProtKB:P55286",
  "gene_name": "Cadherin-8",
  "term_label": "adherens junction",
  "gene_symbol": "CDH8",
  "term_id": "GO:0005912"
}